regulation of response to DNA integrity checkpoint signaling [GO:1902151] (biological process) Also known as: regulation of DNA integrity checkpoint effector process, regulation of response to signal involved in DNA integrity checkpoint Sources: GOC:TermGenie, GOC:mtg_cell_cycle Relationships: is a type of GO:1902145; regulates response to DNA integrity checkpoint signaling [GO:0072402] Subtypes: GO:1902152, regulation of response to DNA damage checkpoint signaling [GO:1902153] Definition: Any process that modulates the frequency, rate or extent of response to DNA integrity checkpoint signaling.